membrane coat [GO:0030117] (cellular component) Definition: Any of several different proteinaceous coats that can associate with membranes. Membrane coats include those formed by clathrin plus an adaptor complex, the COPI and COPII complexes, and possibly others. They are found associated with membranes on many vesicles as well as other membrane features such as pits and perhaps tubules. Subtypes: clathrin coat [GO:0030118], vesicle coat [GO:0030120] Relationships: is a type of GO:0098796; is part of cytoplasm [GO:0005737]; is part of coated membrane [GO:0048475] Sources: GOC:mah